AV node cell-bundle of His cell adhesion involved in cell communication [GO:0086072] (biological process) Relationships: is a type of GO:0034113; is_a GO:0086042; BFO_0000050 GO:0086067 Definition: The attachment of an AV node cell to an bundle of His cell via adhesion molecules that results in the cells being juxtaposed so that they can communicate. Also known as: atrioventricular node cell-bundle of His cell adhesion involved in cell communication Sources: GOC:BHF, GOC:mtg_cardiac_conduct_nov11